histone H2BS36 kinase activity [GO:0140823] (molecular function) Definition: Catalysis of the reaction: histone H2B-serine (position 36) + ATP = histone H2B-phosphoserine (position 36) + ADP. This reaction is the addition of a phosphate group to the serine residue at position 36 of histone H2B. Also known as: histone H2B-S36 kinase activity, histone kinase activity (H2B-S36 specific) Relationships: is a type of protein serine/threonine kinase activity [GO:0004674]; is a type of histone H2B kinase activity [GO:0140998] References: PMID:32822587 Note: Note that the residue position corresponds to the canonical human H2B histone (UniProtKB:P62807); this residue is conserved across all animals, and is replaced by a Thr in plants and fungi, but seems to be missing from Dictyostelium. Residue 1 is the first residue following removal of the initiating Methionine (Met). Note that each histone is encoded by multiple genes, and sequences may vary across different genes within an organism.